metanephric long descending thin limb development [GO:0072269] (biological process) Definition: The process whose specific outcome is the progression of the metanephric long descending thin limb over time, from its formation to the mature structure. The metanephric long descending thin limb is the descending thin limb of a long nephron in the metanephros that has a squamous epithelial morphology. The long descending limb starts in the inner stripe of the outer medulla and extends into the inner medulla. Sources: GOC:mtg_kidney_jan10 Relationships: is_a GO:0072064; is a type of metanephric nephron epithelium development [GO:0072243]; is part of metanephric long nephron development [GO:0072238]